{
  "gene_symbol": "SLC30A8",
  "gene": "UniProtKB:Q8IWU4",
  "gene_name": "Proton-coupled zinc antiporter SLC30A8",
  "term_label": "zinc ion transmembrane transport",
  "term_id": "GO:0071577"
}